{
  "term_label": "extracellular matrix structural constituent",
  "term_id": "GO:0005201",
  "gene": "UniProtKB:Q12805",
  "gene_symbol": "EFEMP1",
  "gene_name": "EGF-containing fibulin-like extracellular matrix protein 1"
}